{
  "term_id": "GO:0005770",
  "term_label": "late endosome",
  "gene": "UniProtKB:Q2KHT3",
  "gene_name": "Protein CLEC16A",
  "gene_symbol": "CLEC16A"
}